organelle outer membrane [GO:0031968] (cellular component) Definition: The outer, i.e. cytoplasm-facing in a cellular organelle, lipid bilayer of an organelle envelope. Sources: GOC:mah Relationships: is a type of GO:0019867; is a type of GO:0098588; is part of organelle envelope [GO:0031967] Subtypes: nuclear outer membrane [GO:0005640], mitochondrial outer membrane [GO:0005741], plastid outer membrane [GO:0009527], chloroplast thylakoid membrane [GO:0009535]